{
  "gene": "UniProtKB:Q8TDH9",
  "term_label": "Unknown biological process",
  "term_id": "UNKNOWN:0002",
  "gene_symbol": "BLOC1S5",
  "gene_name": "Biogenesis of lysosome-related organelles complex 1 subunit 5"
}